{
  "gene": "UniProtKB:O60341",
  "term_id": "GO:0000785",
  "gene_symbol": "KDM1A",
  "gene_name": "Lysine-specific histone demethylase 1A",
  "term_label": "chromatin"
}